{
  "gene_name": "NT-3 growth factor receptor",
  "gene_symbol": "NTRK3",
  "gene": "UniProtKB:Q16288",
  "term_id": "GO:1990090",
  "term_label": "cellular response to nerve growth factor stimulus"
}